{
  "gene": "UniProtKB:Q5VWX1",
  "gene_symbol": "KHDRBS2",
  "term_label": "mRNA binding",
  "gene_name": "KH domain-containing, RNA-binding, signal transduction-associated protein 2",
  "term_id": "GO:0003729"
}